{
  "term_label": "immunoglobulin receptor binding",
  "gene_symbol": "IGHG3",
  "gene": "UniProtKB:P01860",
  "gene_name": "Immunoglobulin heavy constant gamma 3",
  "term_id": "GO:0034987"
}